inositol phosphate catabolic process [GO:0071545] (biological process) Also known as: inositol phosphate breakdown, inositol phosphate catabolism, inositol phosphate degradation, myo-inositol phosphate catabolic process Definition: The chemical reactions and pathways resulting in the breakdown of an inositol phosphate, 1,2,3,4,5,6-cyclohexanehexol, with one or more phosphate groups attached. Sources: GOC:mah Relationships: is a type of inositol phosphate metabolic process [GO:0043647]; is a type of polyol catabolic process [GO:0046174]; is a type of organophosphate catabolic process [GO:0046434] Subtypes: diphosphoinositol polyphosphate catabolic process [GO:0071544]